{
  "term_label": "UDP phosphatase activity",
  "gene": "UniProtKB:Q8WVQ1",
  "term_id": "GO:0045134",
  "gene_name": "Soluble calcium-activated nucleotidase 1",
  "gene_symbol": "CANT1"
}